{
  "term_label": "protein polyubiquitination",
  "gene_name": "Putative ubiquitin-conjugating enzyme E2 N-like",
  "gene": "UniProtKB:Q5JXB2",
  "gene_symbol": "UBE2NL",
  "term_id": "GO:0000209"
}